angiogenesis involved in coronary vascular morphogenesis [GO:0060978] (biological process) Also known as: angiogenesis involved in cardiac vascular morphogenesis, angiogenesis involved in heart vascular morphogenesis, coronary blood vessel angiogenesis, coronary vasculature angiogenesis Relationships: is a type of angiogenesis [GO:0001525]; is part of coronary vasculature morphogenesis [GO:0060977] Definition: Blood vessel formation in the heart when new vessels emerge from the proliferation of pre-existing blood vessels. Sources: GOC:mtg_heart